{
  "gene_symbol": "GIGYF2",
  "gene": "UniProtKB:Q6Y7W6",
  "term_label": "proximal dendrite",
  "gene_name": "GRB10-interacting GYF protein 2",
  "term_id": "GO:1990635"
}